{
  "gene": "UniProtKB:P12644",
  "term_label": "positive regulation of cell population proliferation",
  "gene_name": "Bone morphogenetic protein 4",
  "gene_symbol": "BMP4",
  "term_id": "GO:0008284"
}